{
  "gene_symbol": "ADA",
  "term_id": "GO:0009897",
  "gene": "UniProtKB:P00813",
  "gene_name": "Adenosine deaminase",
  "term_label": "external side of plasma membrane"
}